{
  "gene_name": "Zinc finger protein 843",
  "gene_symbol": "ZNF843",
  "term_id": "UNKNOWN:0001",
  "gene": "UniProtKB:Q8N446",
  "term_label": "Unknown molecular function"
}